{
  "gene_name": "Chemerin-like receptor 2",
  "gene_symbol": "CMKLR2",
  "gene": "UniProtKB:P46091",
  "term_label": "G protein-coupled receptor activity",
  "term_id": "GO:0004930"
}